negative regulation of DNA recombinase disassembly [GO:0062110] (biological process) Definition: Any process that stops, prevents, or reduces the frequency, rate or extent of DNA recombinase complex disassembly, the disaggregation of a DNA recombinase complex into its constituent components. Relationships: is a type of negative regulation of protein-containing complex disassembly [GO:0043242]; is a type of GO:0062109; negatively regulates DNA recombinase disassembly [GO:1990986] References: PMID:30297419